{
  "term_label": "Unknown molecular function",
  "gene": "UniProtKB:Q96M15",
  "gene_symbol": "IGF2BP2-AS1",
  "term_id": "UNKNOWN:0001",
  "gene_name": "Putative uncharacterized protein IGF2BP2-AS1"
}